negative regulation of metanephric comma-shaped body morphogenesis [GO:2000007] (biological process) Sources: GOC:mtg_kidney_jan10, GOC:obol, GOC:yaf Definition: Any process that stops, prevents, or reduces the frequency, rate or extent of metanephric comma-shaped body morphogenesis. Relationships: is_a negative regulation of developmental process [GO:0051093]; is a type of GO:2000006; negatively regulates metanephric comma-shaped body morphogenesis [GO:0072278]